{
  "term_label": "COPI coating of Golgi vesicle",
  "gene_symbol": "ARFGAP3",
  "term_id": "GO:0048205",
  "gene": "UniProtKB:Q9NP61",
  "gene_name": "ADP-ribosylation factor GTPase-activating protein 3"
}